{
  "gene": "UniProtKB:Q99973",
  "gene_symbol": "TEP1",
  "gene_name": "Telomerase protein component 1",
  "term_label": "telomere maintenance via recombination",
  "term_id": "GO:0000722"
}